{
  "gene_name": "Isochorismatase domain-containing protein 1",
  "term_id": "UNKNOWN:0002",
  "gene": "UniProtKB:Q96CN7",
  "term_label": "Unknown biological process",
  "gene_symbol": "ISOC1"
}